hepatocyte growth factor receptor activity [GO:0005008] (molecular function) Relationships: is a type of GO:0004714; is part of hepatocyte growth factor receptor signaling pathway [GO:0048012]; has part hepatocyte growth factor binding [GO:0036458] Definition: Combining with hepatocyte growth factor receptor ligand and transmitting the signal across the plasma membrane to initiate a change in cell activity. Note: Note that this term represents an activity and not a gene product, and should only be used when the receptor binds the ligand HGF. For receptors that bind other growth factors, consider annotating to other terms under 'transmembrane signaling receptor activity ; GO:0004888. Also known as: HGF receptor activity, HGF-activated receptor activity, hepatocyte growth factor-activated receptor activity Sources: GOC:mah